{
  "gene_name": "Putative signal peptidase complex catalytic subunit SEC11B",
  "term_id": "GO:0008233",
  "gene_symbol": "SEC11B",
  "gene": "UniProtKB:P0C7V7",
  "term_label": "peptidase activity"
}